{
  "gene": "UniProtKB:Q9NRX2",
  "term_label": "Unknown biological process",
  "term_id": "UNKNOWN:0002",
  "gene_name": "Large ribosomal subunit protein bL17m",
  "gene_symbol": "MRPL17"
}